{
  "term_label": "antiviral innate immune response",
  "term_id": "GO:0140374",
  "gene_symbol": "OAS1",
  "gene": "UniProtKB:P00973",
  "gene_name": "2'-5'-oligoadenylate synthase 1"
}